response to G1 cell size control checkpoint signaling [GO:0072449] (biological process) Relationships: is a type of GO:0072470 Definition: A process that occurs in response to signals generated as a result of mitotic cell cycle G1/S transition size control checkpoint signaling. Sources: GOC:mtg_cell_cycle Also known as: mitotic cell cycle G1/S transition size control checkpoint effector process, response to signal involved in mitotic cell cycle G1/S transition size control checkpoint